{
  "term_label": "cell migration",
  "gene": "UniProtKB:Q8IVF7",
  "term_id": "GO:0016477",
  "gene_symbol": "FMNL3",
  "gene_name": "Formin-like protein 3"
}